endocytosed synaptic vesicle processing via endosome [GO:0099592] (biological process) Relationships: is a type of vesicle-mediated transport in synapse [GO:0099003]; is a type of GO:0099532; is part of synaptic vesicle recycling via endosome [GO:0036466] Sources: GOC:dos Definition: The process in which endocytosed synaptic vesicles fuse to the presynaptic endosome followed by sorting of synaptic vesicle components and budding of new synaptic vesicles. Also known as: synaptic vesicle processing via endosome involved in synaptic vesicle recycling